{
  "term_label": "olfactory receptor activity",
  "gene_name": "Olfactory receptor 1A1",
  "gene": "UniProtKB:Q9P1Q5",
  "gene_symbol": "OR1A1",
  "term_id": "GO:0004984"
}